{
  "term_label": "Unknown biological process",
  "gene": "UniProtKB:Q9BSH4",
  "gene_name": "Translational activator of cytochrome c oxidase 1",
  "gene_symbol": "TACO1",
  "term_id": "UNKNOWN:0002"
}